{
  "gene_symbol": "GPSM2",
  "gene": "UniProtKB:P81274",
  "gene_name": "G-protein-signaling modulator 2",
  "term_label": "cell cortex",
  "term_id": "GO:0005938"
}